{
  "gene": "UniProtKB:Q8TAG6",
  "gene_name": "Vexin",
  "term_label": "Unknown cellular component",
  "term_id": "UNKNOWN:0003",
  "gene_symbol": "VXN"
}